{
  "term_id": "UNKNOWN:0003",
  "gene_name": "Glutaminase liver isoform, mitochondrial",
  "gene_symbol": "GLS2",
  "term_label": "Unknown cellular component",
  "gene": "UniProtKB:Q9UI32"
}